{
  "gene_name": "Carboxypeptidase N catalytic chain",
  "gene": "UniProtKB:P15169",
  "term_label": "peptide metabolic process",
  "gene_symbol": "CPN1",
  "term_id": "GO:0006518"
}